{
  "gene_symbol": "PRPF40B",
  "term_label": "U2-type prespliceosome",
  "gene": "UniProtKB:Q6NWY9",
  "term_id": "GO:0071004",
  "gene_name": "Pre-mRNA-processing factor 40 homolog B"
}